{
  "gene_symbol": "GRK1",
  "term_label": "regulation of signal transduction",
  "gene_name": "Rhodopsin kinase GRK1",
  "term_id": "GO:0009966",
  "gene": "UniProtKB:Q15835"
}